pronephric nephron tubule development [GO:0039020] (biological process) Relationships: is_a nephron tubule development [GO:0072080]; is part of GO:0039019 Subtypes: pronephric proximal tubule development [GO:0035776], GO:0035777 Definition: The process whose specific outcome is the progression of a pronephric nephron tubule over time, from its formation to the mature structure. The pronephric nephron tubule is an epithelial tube that is part of the pronephric nephron and connects the filtration unit (glomerulus or glomus) of the pronephros to the pronephric duct. References: PMID:19909807, PMID:9268568 Sources: GOC:mtg_kidney_jan10 Regulation: regulated by regulation of pronephric nephron tubule development [GO:1900206]; negatively regulated by negative regulation of pronephric nephron tubule development [GO:1900207]